{
  "term_id": "UNKNOWN:0001",
  "gene_symbol": "MORN2",
  "gene_name": "MORN repeat-containing protein 2",
  "gene": "UniProtKB:Q502X0",
  "term_label": "Unknown molecular function"
}